{
  "gene_symbol": "ISCU",
  "gene_name": "Iron-sulfur cluster assembly enzyme ISCU",
  "gene": "UniProtKB:Q9H1K1",
  "term_id": "GO:0008198",
  "term_label": "ferrous iron binding"
}